{
  "term_label": "nuclear pore",
  "gene_name": "RANBP2-like and GRIP domain-containing protein 8",
  "term_id": "GO:0005643",
  "gene_symbol": "RGPD8",
  "gene": "UniProtKB:O14715"
}